{
  "gene_name": "Protein phosphatase 3 catalytic subunit alpha",
  "term_id": "GO:0033192",
  "gene": "UniProtKB:Q08209",
  "gene_symbol": "PPP3CA",
  "term_label": "calmodulin-dependent protein phosphatase activity"
}